{
  "gene_symbol": "ADPRS",
  "gene": "UniProtKB:Q9NX46",
  "term_id": "GO:0071451",
  "term_label": "cellular response to superoxide",
  "gene_name": "ADP-ribosylhydrolase ARH3"
}